{
  "gene_name": "Zinc finger CCHC domain-containing protein 17",
  "gene": "UniProtKB:Q9NP64",
  "term_id": "GO:0003723",
  "gene_symbol": "ZCCHC17",
  "term_label": "RNA binding"
}